actin cortical patch organization [GO:0044396] (biological process) Also known as: actin cortical patch organisation Relationships: is a type of cellular component organization [GO:0016043]; is part of GO:0030866 Definition: A process that is carried out at the cellular level and results in the assembly, arrangement of constituent parts, or disassembly of an actin cortical patch, a discrete actin-containing structure found at the plasma membrane in cells, at sites of endocytosis. Sources: GOC:jl Subtypes: actin cortical patch assembly [GO:0000147]